{
  "term_label": "cellular response to oxidative stress",
  "term_id": "GO:0034599",
  "gene_symbol": "SRXN1",
  "gene": "UniProtKB:Q9BYN0",
  "gene_name": "Sulfiredoxin-1"
}